regulation of branching involved in salivary gland morphogenesis by extracellular matrix-epithelial cell signaling [GO:0060668] (BP) Definition: Any process that modulates the rate, frequency, or extent of salivary gland branching as a result of the transfer of information from the extracellular matrix to the epithelium of the salivary gland. Also known as: regulation of branching involved in salivary gland morphogenesis by extracellular matrix-epithelial cell signalling Sources: GOC:dph Relationships: is a type of extracellular matrix-cell signaling [GO:0035426]; is a type of regulation of branching involved in salivary gland morphogenesis [GO:0060693]